{
  "term_id": "GO:0008494",
  "term_label": "translation activator activity",
  "gene_symbol": "DAZL",
  "gene_name": "Deleted in azoospermia-like",
  "gene": "UniProtKB:Q92904"
}